transmembrane receptor protein tyrosine kinase activity [GO:0004714] (molecular function) Definition: Combining with a signal and transmitting the signal from one side of the membrane to the other to initiate a change in cell activity by catalysis of the reaction: ATP + a protein-L-tyrosine = ADP + a protein-L-tyrosine phosphate. Also known as: receptor protein tyrosine kinase activity, receptor protein-tyrosine kinase activity Relationships: is a type of protein tyrosine kinase activity [GO:0004713]; is a type of transmembrane receptor protein kinase activity [GO:0019199] Regulation: negatively regulated by GO:0030293; positively regulated by transmembrane receptor protein tyrosine kinase activator activity [GO:0030297] Subtypes: GO:0005003, epidermal growth factor receptor activity [GO:0005006], fibroblast growth factor receptor activity [GO:0005007], hepatocyte growth factor receptor activity [GO:0005008], GO:0005009, GO:0005010, macrophage colony-stimulating factor receptor activity [GO:0005011], platelet-derived growth factor receptor activity [GO:0005017], stem cell factor receptor activity [GO:0005020], vascular endothelial growth factor receptor activity [GO:0005021], boss receptor activity [GO:0008288], placental growth factor receptor activity [GO:0036332], protein tyrosine kinase collagen receptor activity [GO:0038062], brain-derived neurotrophic factor receptor activity [GO:0060175] Sources: EC:2.7.10.1, GOC:mah